{
  "gene_name": "Glutathione S-transferase Mu 4",
  "term_id": "GO:0006749",
  "gene": "UniProtKB:Q03013",
  "term_label": "glutathione metabolic process",
  "gene_symbol": "GSTM4"
}